{
  "gene_symbol": "TIMP4",
  "gene_name": "Metalloproteinase inhibitor 4",
  "gene": "UniProtKB:Q99727",
  "term_id": "GO:0031012",
  "term_label": "extracellular matrix"
}